{
  "term_id": "GO:0035091",
  "term_label": "phosphatidylinositol binding",
  "gene_name": "Phosphatidylinositol transfer protein alpha isoform",
  "gene_symbol": "PITPNA",
  "gene": "UniProtKB:Q00169"
}